{
  "gene": "UniProtKB:O95070",
  "gene_symbol": "YIF1A",
  "gene_name": "Protein YIF1A",
  "term_label": "Golgi membrane",
  "term_id": "GO:0000139"
}